positive regulation of peptidase activity [GO:0010952] (biological process) Relationships: is a type of GO:0045862; is_a positive regulation of hydrolase activity [GO:0051345]; is a type of regulation of peptidase activity [GO:0052547]; positively regulates peptidase activity [GO:0008233] Sources: GOC:dph, GOC:tb Subtypes: positive regulation of endopeptidase activity [GO:0010950], positive regulation of metallopeptidase activity [GO:1905050], positive regulation of aspartic-type peptidase activity [GO:1905247], positive regulation of ubiquitin-specific protease activity [GO:2000158] Definition: Any process that increases the frequency, rate or extent of peptidase activity, the hydrolysis of peptide bonds within proteins.